{
  "gene_symbol": "PPP1R3E",
  "gene_name": "Protein phosphatase 1 regulatory subunit 3E",
  "gene": "UniProtKB:Q9H7J1",
  "term_id": "GO:0000164",
  "term_label": "protein phosphatase type 1 complex"
}